{
  "gene_name": "Zinc finger protein 654",
  "gene_symbol": "ZNF654",
  "term_label": "DNA binding",
  "term_id": "GO:0003677",
  "gene": "UniProtKB:Q8IZM8"
}